{
  "term_label": "amyloid-beta binding",
  "gene": "UniProtKB:Q9BX74",
  "term_id": "GO:0001540",
  "gene_name": "TM2 domain-containing protein 1",
  "gene_symbol": "TM2D1"
}